cell-cell adhesion involved in mesendodermal cell migration [GO:0003370] (biological process) Relationships: is a type of GO:0003367; is a type of cell-cell adhesion involved in gastrulation [GO:0070586]; is part of establishment of cell polarity involved in mesendodermal cell migration [GO:0003369] Sources: GOC:ascb_2009, GOC:dph, GOC:tb Definition: The attachment of mesendodermal cells to each other that contributes to the establishment of cell polarity that is part of the directed movement of the cells of the mesendoderm.